{
  "gene_symbol": "PYCARD-AS1",
  "term_id": "UNKNOWN:0002",
  "term_label": "Unknown biological process",
  "gene": "UniProtKB:I3L0S3",
  "gene_name": "Putative uncharacterized protein PYCARD-AS1"
}